ABC-type D-galactofuranose transporter [GO:0103116] (molecular function) Also known as: ATP-dependent alpha-D-galactofuranose transporter activity, alpha-D-galactofuranose transporter activity, ATPase-coupled alpha-D-galactofuranose transporter activity Relationships: is a type of galactose transmembrane transporter activity [GO:0005354]; is_a ABC-type monosaccharide transporter activity [GO:0015407]; is part of GO:0042875 References: PMID:19744923 Sources: GOC:pz, RHEA:61716 Definition: Catalysis of the reaction: alpha-D-galactofuranose + ATP + H2O = alpha-D-galactofuranose + hydrogenphosphate + ADP + H+.